regulation of detection of mechanical stimulus involved in sensory perception of touch [GO:1905787] (biological process) Subtypes: negative regulation of detection of mechanical stimulus involved in sensory perception of touch [GO:1905788], GO:1905789 Also known as: regulation of perception of touch, detection of mechanical stimulus, regulation of perception of touch, sensory detection of mechanical stimulus, regulation of perception of touch, sensory transduction of mechanical stimulus, regulation of sensory detection of mechanical stimulus during perception of touch, regulation of sensory transduction of mechanical stimulus during perception of touch, regulation of tactition, sensory detection of mechanical stimulus Relationships: is a type of regulation of response to external stimulus [GO:0032101]; is a type of regulation of sensory perception [GO:0051931]; regulates detection of mechanical stimulus involved in sensory perception of touch [GO:0050976] Definition: Any process that modulates the frequency, rate or extent of detection of mechanical stimulus involved in sensory perception of touch. References: PMID:8692859 Sources: GOC:TermGenie, GO_REF:0000058